{
  "gene_name": "Ephrin type-A receptor 10",
  "gene_symbol": "EPHA10",
  "gene": "UniProtKB:Q5JZY3",
  "term_id": "GO:0030425",
  "term_label": "dendrite"
}